post-embryonic animal morphogenesis [GO:0009886] (biological process) Subtypes: establishment of imaginal disc-derived wing hair orientation [GO:0001737], GO:0007436, apposition of dorsal and ventral imaginal disc-derived wing surfaces [GO:0007475], tergite morphogenesis [GO:0007490], GO:0007491, imaginal disc eversion [GO:0007561], imaginal disc-derived wing vein morphogenesis [GO:0008586], imaginal disc-derived wing margin morphogenesis [GO:0008587], proboscis morphogenesis, labial disc-derived [GO:0010782], proboscis morphogenesis, eye-antennal disc-derived [GO:0010783], proboscis morphogenesis, clypeo-labral disc-derived [GO:0010784], GO:0016335, GO:0016348, GO:0035070, GO:0035120, GO:0035193, GO:0035318, imaginal disc-derived wing hair elongation [GO:0035319], post-embryonic body morphogenesis [GO:0040032], imaginal disc fusion [GO:0046528], imaginal disc fusion, thorax closure [GO:0046529], post-embryonic ectodermal digestive tract morphogenesis [GO:0048614], post-embryonic anterior midgut (ectodermal) morphogenesis [GO:0048616], post-embryonic foregut morphogenesis [GO:0048618], post-embryonic hindgut morphogenesis [GO:0048620], post-embryonic digestive tract morphogenesis [GO:0048621], instar larval or pupal morphogenesis [GO:0048707], labrum morphogenesis [GO:0048716], anterior cibarial plate morphogenesis [GO:0048717], epistomal sclerite morphogenesis [GO:0048719], GO:0048720, clypeus morphogenesis [GO:0048721], GO:0048800, antennal joint morphogenesis [GO:0048801], notum morphogenesis [GO:0048802], analia morphogenesis [GO:0048809], ocellus morphogenesis [GO:0048816], post-embryonic retina morphogenesis in camera-type eye [GO:0060060], GO:0090253, GO:0090254 Relationships: is a type of anatomical structure morphogenesis [GO:0009653]; is part of GO:0009791 Also known as: post-embryonic morphogenesis of an anatomical structure Sources: GOC:go_curators Definition: The process, occurring after animal embryonic development, by which anatomical structures are generated and organized.